{
  "term_id": "UNKNOWN:0001",
  "gene_name": "RELT-like protein 1",
  "term_label": "Unknown molecular function",
  "gene_symbol": "RELL1",
  "gene": "UniProtKB:Q8IUW5"
}